reverse transcription [GO:0001171] (biological process) References: PMID:20358252 Sources: GOC:txnOH Regulation: regulated by regulation of reverse transcription [GO:1900268]; negatively regulated by negative regulation of reverse transcription [GO:1900269]; positively regulated by positive regulation of reverse transcription [GO:1900270] Relationships: is a type of GO:0006278; BFO_0000051 RNA-directed DNA polymerase activity [GO:0003964]; has part exoribonuclease H activity [GO:0004533] Definition: A DNA synthesis process that uses RNA as the initial template for synthesis of DNA, but which also includes an RNase activity to remove the RNA strand of an RNA-DNA heteroduplex produced by the RNA-dependent synthesis step and use of the initial DNA strand as a template for DNA synthesis.